{
  "term_id": "GO:0034967",
  "gene_symbol": "SETD5",
  "gene_name": "Histone-lysine N-methyltransferase SETD5",
  "term_label": "Set3 complex",
  "gene": "UniProtKB:Q9C0A6"
}